{
  "gene": "UniProtKB:Q1HG44",
  "gene_symbol": "DUOXA2",
  "term_label": "membrane",
  "term_id": "GO:0016020",
  "gene_name": "Dual oxidase maturation factor 2"
}